{
  "gene_name": "Keratin-associated protein 19-8",
  "gene": "UniProtKB:Q3LI54",
  "term_label": "Unknown cellular component",
  "term_id": "UNKNOWN:0003",
  "gene_symbol": "KRTAP19-8"
}